{
  "gene_name": "Bridge-like lipid transfer protein family member 3B",
  "term_label": "Unknown cellular component",
  "gene": "UniProtKB:A0JNW5",
  "term_id": "UNKNOWN:0003",
  "gene_symbol": "BLTP3B"
}